{
  "gene_symbol": "GBX1",
  "gene": "UniProtKB:Q14549",
  "gene_name": "Homeobox protein GBX-1",
  "term_label": "RNA polymerase II transcription regulatory region sequence-specific DNA binding",
  "term_id": "GO:0000977"
}